{
  "gene_symbol": "H2BC21",
  "term_label": "nucleosome",
  "gene_name": "Histone H2B type 2-E",
  "term_id": "GO:0000786",
  "gene": "UniProtKB:Q16778"
}